{
  "gene_name": "T cell receptor alpha variable 27",
  "term_id": "UNKNOWN:0003",
  "term_label": "Unknown cellular component",
  "gene_symbol": "TRAV27",
  "gene": "UniProtKB:A0A087WT01"
}